{
  "gene": "UniProtKB:O95340",
  "gene_symbol": "PAPSS2",
  "term_id": "UNKNOWN:0003",
  "gene_name": "Bifunctional 3'-phosphoadenosine 5'-phosphosulfate synthase 2",
  "term_label": "Unknown cellular component"
}